{
  "gene": "UniProtKB:Q8NCK3",
  "gene_symbol": "ZNF485",
  "gene_name": "Zinc finger protein 485",
  "term_label": "DNA-binding transcription activator activity, RNA polymerase II-specific",
  "term_id": "GO:0001228"
}